interleukin-21 receptor binding [GO:0001531] (molecular function) Definition: Binding to an interleukin-21 receptor. Relationships: is a type of cytokine receptor binding [GO:0005126] Sources: GOC:ai Also known as: IL-21, interleukin-21 receptor ligand